negative regulation of DNA recombination at telomere [GO:0048239] (biological process) Relationships: is a type of negative regulation of DNA recombination [GO:0045910]; is a type of regulation of DNA recombination at telomere [GO:0072695] Also known as: down regulation of telomeric recombination at telomere, down-regulation of telomeric recombination at telomere, downregulation of telomeric recombination at telomere, negative regulation of telomeric recombination at telomere, suppression of telomeric recombination at telomere, inhibition of telomeric recombination at telomere References: PMID:9635193 Sources: GOC:jid Definition: Any process that stops, prevents, or reduces the frequency, rate or extent of genetic recombination within the telomere. Subtypes: negative regulation of telomere maintenance via recombination [GO:0032208]